response to lectin [GO:1990840] (biological process) Note: This term refers to endogenous (evolved) responses to lectins (endogenous or exogenous), it does not cover the events that happen due to lectin toxicity. Subtypes: cellular response to lectin [GO:1990858] Relationships: is a type of response to biotic stimulus [GO:0009607] References: PMID:25996210, PMID:26306444 Definition: Any process that results in a change in state or activity of a cell or an organism (in terms of movement, secretion, enzyme production, gene expression, etc.) as a result of a lectin stimulus. A lectin is a carbohydrate-binding protein, highly specific for binding sugar moieties.